{
  "term_label": "cytosol",
  "term_id": "GO:0005829",
  "gene_symbol": "HELZ",
  "gene": "UniProtKB:P42694",
  "gene_name": "Probable helicase with zinc finger domain"
}